{
  "term_label": "Unknown molecular function",
  "gene": "UniProtKB:P00451",
  "gene_name": "Coagulation factor VIII",
  "gene_symbol": "F8",
  "term_id": "UNKNOWN:0001"
}